{
  "term_id": "GO:0014069",
  "gene": "UniProtKB:Q86SQ6",
  "term_label": "postsynaptic density",
  "gene_symbol": "ADGRA1",
  "gene_name": "Adhesion G protein-coupled receptor A1"
}